{
  "gene_symbol": "EGLN2",
  "term_label": "peptidyl-proline 4-dioxygenase activity",
  "gene": "UniProtKB:Q96KS0",
  "term_id": "GO:0031545",
  "gene_name": "Prolyl hydroxylase EGLN2"
}